negative regulation of cellular response to gamma radiation [GO:1905844] (biological process) Definition: Any process that stops, prevents or reduces the frequency, rate or extent of cellular response to gamma radiation. Also known as: down regulation of cellular response to gamma radiation, down-regulation of cellular response to gamma radiation, downregulation of cellular response to gamma radiation, inhibition of cellular response to gamma radiation, down regulation of cellular response to gamma ray, down regulation of cellular response to gamma-ray photon, down-regulation of cellular response to gamma ray, down-regulation of cellular response to gamma-ray photon, downregulation of cellular response to gamma ray, downregulation of cellular response to gamma-ray photon, inhibition of cellular response to gamma ray, inhibition of cellular response to gamma-ray photon, negative regulation of cellular response to gamma ray, negative regulation of cellular response to gamma-ray photon Relationships: is a type of GO:0048523; is a type of regulation of cellular response to gamma radiation [GO:1905843]; is a type of negative regulation of response to gamma radiation [GO:2001229]; negatively regulates cellular response to gamma radiation [GO:0071480] References: PMID:23505386 Sources: GOC:TermGenie, GO_REF:0000058